{
  "term_id": "GO:0005923",
  "gene_name": "Tight junction protein ZO-1",
  "gene": "UniProtKB:Q07157",
  "gene_symbol": "TJP1",
  "term_label": "bicellular tight junction"
}